{
  "gene_symbol": "TTC23",
  "term_id": "UNKNOWN:0003",
  "gene": "UniProtKB:Q5W5X9",
  "term_label": "Unknown cellular component",
  "gene_name": "Tetratricopeptide repeat protein 23"
}